stereocilium tip [GO:0032426] (cellular component) References: PMID:17021180, PMID:27565685 Sources: GOC:ecd, GOC:krc Relationships: is a type of GO:0110165; is part of stereocilium [GO:0032420] Definition: A distinct compartment at the tip of a stereocilium, distal to the site of attachment to the apical cell surface. It consists of a dense matrix bridging the barbed ends of the stereocilium actin filaments with the overlying plasma membrane, is dynamic compared to the shaft, and is required for stereocilium elongation.